rDNA heterochromatin [GO:0033553] (cellular component) Relationships: is a type of GO:0000792 References: PMID:20661445 Sources: GOC:mah Also known as: ribosomal DNA heterochromatin, nuclear rDNA heterochromatin, ribosomal DNA heterochromatin of cell nucleus, ribosomal DNA heterochromatin of nucleus Definition: A region of heterochromatin located at the rDNA repeats in a chromosome.